{
  "gene_name": "Actin, cytoplasmic 2",
  "term_id": "GO:0005884",
  "gene": "UniProtKB:P63261",
  "term_label": "actin filament",
  "gene_symbol": "ACTG1"
}